laminin-3 complex [GO:0005608] (CC) Definition: A laminin complex composed of alpha1, beta2 and gamma1 polypeptide chains. Sources: MEDLINE:95005761 Also known as: laminin-121 complex Relationships: is a type of laminin complex [GO:0043256]